{
  "gene": "UniProtKB:Q53TN4",
  "term_label": "Unknown biological process",
  "gene_symbol": "CYBRD1",
  "gene_name": "Plasma membrane ascorbate-dependent reductase CYBRD1",
  "term_id": "UNKNOWN:0002"
}